{
  "term_label": "cell chemotaxis",
  "term_id": "GO:0060326",
  "gene_name": "Defensin beta 4A",
  "gene_symbol": "DEFB4B",
  "gene": "UniProtKB:O15263"
}